{
  "gene_symbol": "A0A2R8YCY7",
  "gene": "UniProtKB:A0A2R8YCY7",
  "gene_name": "Immunoglobulin subtype domain-containing protein",
  "term_id": "GO:0005886",
  "term_label": "plasma membrane"
}